{
  "gene_name": "Insulin-like growth factor 2 mRNA-binding protein 3",
  "term_label": "CRD-mediated mRNA stabilization",
  "gene": "UniProtKB:O00425",
  "gene_symbol": "IGF2BP3",
  "term_id": "GO:0070934"
}